{
  "gene_symbol": "RYR1",
  "term_id": "GO:0030018",
  "gene_name": "Ryanodine receptor 1",
  "gene": "UniProtKB:P21817",
  "term_label": "Z disc"
}